{
  "term_label": "Unknown molecular function",
  "gene_name": "EF-hand calcium-binding domain-containing protein 12",
  "gene_symbol": "EFCAB12",
  "term_id": "UNKNOWN:0001",
  "gene": "UniProtKB:Q6NXP0"
}